{
  "gene": "UniProtKB:Q07687",
  "term_id": "GO:0006357",
  "gene_symbol": "DLX2",
  "term_label": "regulation of transcription by RNA polymerase II",
  "gene_name": "Homeobox protein DLX-2"
}